{
  "term_label": "myofibril",
  "gene": "UniProtKB:Q01449",
  "gene_symbol": "MYL7",
  "term_id": "GO:0030016",
  "gene_name": "Myosin regulatory light chain 2, atrial isoform"
}